{
  "gene_symbol": "AKAP6",
  "gene_name": "A-kinase anchor protein 6",
  "term_label": "sarcoplasmic reticulum",
  "gene": "UniProtKB:Q13023",
  "term_id": "GO:0016529"
}